{
  "term_label": "transmembrane receptor protein tyrosine kinase adaptor activity",
  "gene_name": "SH2B adapter protein 2",
  "gene": "UniProtKB:O14492",
  "gene_symbol": "SH2B2",
  "term_id": "GO:0005068"
}